{
  "gene": "UniProtKB:Q9NPJ1",
  "gene_symbol": "MKKS",
  "gene_name": "Molecular chaperone MKKS",
  "term_label": "Unknown molecular function",
  "term_id": "UNKNOWN:0001"
}